{
  "gene": "UniProtKB:O43808",
  "term_id": "GO:0015217",
  "gene_name": "Peroxisomal membrane protein PMP34",
  "gene_symbol": "SLC25A17",
  "term_label": "ADP transmembrane transporter activity"
}